{
  "gene_name": "tRNA-uridine aminocarboxypropyltransferase 2",
  "term_label": "Unknown cellular component",
  "term_id": "UNKNOWN:0003",
  "gene_symbol": "DTWD2",
  "gene": "UniProtKB:Q8NBA8"
}